{
  "term_label": "nucleus",
  "gene_symbol": "UBE2E3",
  "gene_name": "Ubiquitin-conjugating enzyme E2 E3",
  "term_id": "GO:0005634",
  "gene": "UniProtKB:Q969T4"
}